{
  "term_label": "protein localization to plasma membrane",
  "gene": "UniProtKB:Q86UF1",
  "gene_name": "Tetraspanin-33",
  "gene_symbol": "TSPAN33",
  "term_id": "GO:0072659"
}